{
  "gene_symbol": "CABP5",
  "gene_name": "Calcium-binding protein 5",
  "gene": "UniProtKB:Q9NP86",
  "term_label": "visual perception",
  "term_id": "GO:0007601"
}